{
  "term_id": "GO:0043025",
  "term_label": "neuronal cell body",
  "gene": "UniProtKB:Q13308",
  "gene_symbol": "PTK7",
  "gene_name": "Inactive tyrosine-protein kinase 7"
}